{
  "gene": "UniProtKB:P04350",
  "term_label": "microtubule",
  "gene_name": "Tubulin beta-4A chain",
  "gene_symbol": "TUBB4A",
  "term_id": "GO:0005874"
}